{
  "term_label": "Cul3-RING ubiquitin ligase complex",
  "gene_name": "Influenza virus NS1A-binding protein",
  "gene": "UniProtKB:Q9Y6Y0",
  "term_id": "GO:0031463",
  "gene_symbol": "IVNS1ABP"
}